{
  "gene": "UniProtKB:Q9UKU6",
  "gene_symbol": "TRHDE",
  "gene_name": "Thyrotropin-releasing hormone-degrading ectoenzyme",
  "term_label": "proteolysis",
  "term_id": "GO:0006508"
}